{
  "gene": "UniProtKB:Q86YG4",
  "gene_symbol": "NT5DC4",
  "term_label": "5'-nucleotidase activity",
  "term_id": "GO:0008253",
  "gene_name": "5'-nucleotidase domain-containing protein 4"
}